{
  "gene_symbol": "FAM90A9",
  "term_label": "Unknown biological process",
  "term_id": "UNKNOWN:0002",
  "gene_name": "Putative protein FAM90A9",
  "gene": "UniProtKB:A6NNJ1"
}